vesicle fusion with vacuole [GO:0051469] (biological process) Relationships: is a type of vesicle fusion [GO:0006906]; is a type of vacuole fusion [GO:0097576] Sources: GOC:ai Definition: The joining of the lipid bilayer membrane around a vesicle with the lipid bilayer membrane around the vacuole. Also known as: heterotypic vacuole fusion (non-autophagic), heterotypic vacuole fusion, non-autophagic